{
  "gene_name": "Tyrosine-protein kinase Fes_Fps",
  "term_label": "chemotaxis",
  "gene": "UniProtKB:P07332",
  "gene_symbol": "FES",
  "term_id": "GO:0006935"
}